'de novo' CTP biosynthetic process [GO:0044210] (BP) Relationships: is a type of CTP biosynthetic process [GO:0006241] Also known as: 'de novo' cytidine 5'-triphosphate biosynthetic process Definition: The chemical reactions and pathways resulting in the formation of cytidine 5'-triphosphate (CTP) from simpler components. References: PMID:11912132, PMID:18439916 Sources: GOC:ecd, GOC:jl